{
  "gene_symbol": "POLR2K",
  "term_id": "GO:0005736",
  "term_label": "RNA polymerase I complex",
  "gene": "UniProtKB:P53803",
  "gene_name": "DNA-directed RNA polymerases I, II, and III subunit RPABC4"
}